{
  "gene_symbol": "NOL6",
  "term_id": "UNKNOWN:0001",
  "gene": "UniProtKB:Q9H6R4",
  "gene_name": "Nucleolar protein 6",
  "term_label": "Unknown molecular function"
}